prostaglandin-D synthase activity [GO:0004667] (molecular function) Definition: Catalysis of the reaction: prostaglandin H(2) = prostaglandin D(2). Sources: EC:5.3.99.2, RHEA:10600 Relationships: is a type of GO:0016860 Also known as: (5,13)-(15S)-9alpha,11alpha-epidioxy-15-hydroxyprosta-5,13-dienoate D-isomerase activity, PGD2 synthase activity, PGH-PGD isomerase activity, prostaglandin D2 synthase activity, prostaglandin-H2 D-isomerase activity, prostaglandin-R-prostaglandin D isomerase activity